{
  "term_label": "DNA-binding transcription factor activity, RNA polymerase II-specific",
  "gene": "UniProtKB:P57682",
  "gene_symbol": "KLF3",
  "gene_name": "Krueppel-like factor 3",
  "term_id": "GO:0000981"
}